lutein catabolic process [GO:0062172] (BP) Relationships: is a type of xanthophyll catabolic process [GO:0016124] Definition: The chemical reactions and pathways resulting in the breakdown of lutein. Also known as: lutein breakdown, lutein catabolism, lutein degradation References: PMID:24397433